{
  "term_id": "UNKNOWN:0002",
  "term_label": "Unknown biological process",
  "gene_name": "Proline-rich acidic protein 1",
  "gene_symbol": "PRAP1",
  "gene": "UniProtKB:Q96NZ9"
}